{
  "gene": "UniProtKB:P0DTE4",
  "gene_symbol": "UGT2A1",
  "gene_name": "UDP-glucuronosyltransferase 2A1",
  "term_id": "UNKNOWN:0003",
  "term_label": "Unknown cellular component"
}